{
  "gene": "UniProtKB:Q15024",
  "gene_name": "Exosome complex component RRP42",
  "term_id": "GO:0071035",
  "term_label": "nuclear polyadenylation-dependent rRNA catabolic process",
  "gene_symbol": "EXOSC7"
}